{
  "gene": "UniProtKB:Q8N111",
  "term_id": "GO:0021702",
  "term_label": "cerebellar Purkinje cell differentiation",
  "gene_name": "Cell cycle exit and neuronal differentiation protein 1",
  "gene_symbol": "CEND1"
}